{
  "term_id": "GO:0044325",
  "gene_symbol": "KCNAB3",
  "gene": "UniProtKB:O43448",
  "term_label": "transmembrane transporter binding",
  "gene_name": "Voltage-gated potassium channel subunit beta-3"
}